{
  "gene_symbol": "OR2L5",
  "gene": "UniProtKB:Q8NG80",
  "gene_name": "Olfactory receptor 2L5",
  "term_id": "GO:0004984",
  "term_label": "olfactory receptor activity"
}